{
  "gene_name": "E3 ubiquitin-protein ligase RNF144A",
  "term_label": "ubiquitin-dependent protein catabolic process",
  "gene_symbol": "RNF144A",
  "term_id": "GO:0006511",
  "gene": "UniProtKB:P50876"
}